rhombomere 3 morphogenesis [GO:0021658] (biological process) Definition: The process in which the anatomical structure of rhombomere 3 is generated and organized. Rhombomeres are transverse segments of the developing rhombencephalon. Rhombomeres are lineage restricted, express different genes from one another, and adopt different developmental fates. Rhombomeres are numbered in an anterior to posterior order. Sources: GOC:cls, GOC:curators, GOC:dgh, GOC:dph, GOC:jid Relationships: is a type of rhombomere morphogenesis [GO:0021593]; is part of rhombomere 3 development [GO:0021569]